{
  "gene": "UniProtKB:O95714",
  "term_label": "ubiquitin protein ligase activity",
  "term_id": "GO:0061630",
  "gene_name": "E3 ubiquitin-protein ligase HERC2",
  "gene_symbol": "HERC2"
}